{
  "term_id": "GO:0022602",
  "term_label": "ovulation cycle process",
  "gene_name": "Lutropin-choriogonadotropic hormone receptor",
  "gene_symbol": "LHCGR",
  "gene": "UniProtKB:P22888"
}